{
  "gene_symbol": "SCGB2B2",
  "term_label": "Unknown cellular component",
  "gene_name": "Secretoglobin family 2B member 2",
  "term_id": "UNKNOWN:0003",
  "gene": "UniProtKB:Q4G0G5"
}